{
  "term_id": "GO:0030125",
  "gene": "UniProtKB:Q8TBZ2",
  "gene_name": "MYCBP-associated protein",
  "gene_symbol": "MYCBPAP",
  "term_label": "clathrin vesicle coat"
}